2-iminobutanoate/2-iminopropanoate deaminase [GO:0120241] (molecular function) Note: This enzyme, which has been found in all species and tissues examined, catalyzes the hydrolytic deamination of imine intermediates formed by several types of pyridoxal-5'-phosphate-dependent dehydratases, such as EC 4.3.1.19 and EC 4.3.1.17. The reactions, which can occur spontaneously, are accelerated to minimize the cellular damage that could be caused by these reactive intermediates (from EC:3.5.99.10). Sources: EC:3.5.99.10 Definition: Catalyzes the hydrolytic deamination of imine intermediates formed by several types of pyridoxal-5'-phosphate-dependent dehydratases, such as EC 4.3.1.19 and EC 4.3.1.17. Relationships: is a type of deaminase activity [GO:0019239] Subtypes: 2-iminobutanoate deaminase activity [GO:0120242], 2-iminopropanoate deaminase activity [GO:0120243] Also known as: enamine/imine deaminase, 2-iminobutanoate deaminase, 2-iminopropanoate deaminase, imine intermediate deaminase activity